{
  "gene_name": "Semaphorin-3A",
  "gene": "UniProtKB:Q14563",
  "gene_symbol": "SEMA3A",
  "term_label": "neural crest cell migration",
  "term_id": "GO:0001755"
}